{
  "gene_symbol": "WDR86",
  "gene_name": "WD repeat-containing protein 86",
  "term_label": "Unknown molecular function",
  "gene": "UniProtKB:Q86TI4",
  "term_id": "UNKNOWN:0001"
}